{
  "term_label": "transcription elongation by RNA polymerase II",
  "gene_name": "Transcription elongation factor A N-terminal and central domain-containing protein 2",
  "gene": "UniProtKB:Q96MN5",
  "gene_symbol": "TCEANC2",
  "term_id": "GO:0006368"
}